{
  "gene_name": "Matrix metalloproteinase-16",
  "gene_symbol": "MMP16",
  "term_label": "metalloendopeptidase activity",
  "gene": "UniProtKB:P51512",
  "term_id": "GO:0004222"
}